Langerhans cell chemotaxis [GO:0002409] (biological process) Definition: The movement of a Langerhans cell in response to an external stimulus. References: PMID:16056255, PMID:16387601 Sources: GOC:add Relationships: is a type of myeloid dendritic cell chemotaxis [GO:0002408]